{
  "gene": "UniProtKB:Q156A1",
  "gene_name": "Ataxin-8",
  "term_id": "UNKNOWN:0003",
  "term_label": "Unknown cellular component",
  "gene_symbol": "ATXN8"
}